positive regulation of excitatory synapse assembly [GO:1904891] (biological process) Definition: Any process that activates or increases the frequency, rate or extent of excitatory synapse assembly. Also known as: positive regulation of excitatory synapse formation, up regulation of excitatory synapse assembly, up regulation of excitatory synapse formation, up-regulation of excitatory synapse assembly, up-regulation of excitatory synapse formation, upregulation of excitatory synapse assembly, upregulation of excitatory synapse formation, activation of excitatory synapse assembly, activation of excitatory synapse formation References: PMID:21670302 Sources: GOC:PARL, GOC:TermGenie, GOC:bf, GO_REF:0000058 Relationships: is a type of positive regulation of synapse assembly [GO:0051965]; is a type of regulation of excitatory synapse assembly [GO:1904889]; positively regulates GO:1904861